purine ribonucleoside triphosphate catabolic process [GO:0009207] (biological process) Relationships: is a type of GO:0009146; is a type of ribonucleoside triphosphate catabolic process [GO:0009203]; is a type of purine ribonucleoside triphosphate metabolic process [GO:0009205] Sources: GOC:go_curators, ISBN:0198506732 Also known as: purine ribonucleoside triphosphate breakdown, purine ribonucleoside triphosphate catabolism, purine ribonucleoside triphosphate degradation Subtypes: ITP catabolic process [GO:0006193] Definition: The chemical reactions and pathways resulting in the breakdown of purine ribonucleoside triphosphate, a compound consisting of a purine base linked to a ribose sugar esterified with triphosphate on the sugar.